negative regulation of protein polyglycylation [GO:1903345] (biological process) Relationships: is a type of negative regulation of protein modification process [GO:0031400]; is a type of regulation of protein polyglycylation [GO:1903344]; negatively regulates protein polyglycylation [GO:0018094] Sources: GOC:TermGenie, GOC:sart, GO_REF:0000058 Also known as: down regulation of protein polyglycylation, down-regulation of protein polyglycylation, downregulation of protein polyglycylation, inhibition of protein polyglycylation Definition: Any process that stops, prevents or reduces the frequency, rate or extent of protein polyglycylation.